{
  "gene_symbol": "ZNF358",
  "term_label": "regulation of transcription by RNA polymerase II",
  "gene_name": "Zinc finger protein 358",
  "term_id": "GO:0006357",
  "gene": "UniProtKB:Q9NW07"
}